{
  "gene": "UniProtKB:Q8WUA2",
  "gene_name": "Peptidyl-prolyl cis-trans isomerase-like 4",
  "gene_symbol": "PPIL4",
  "term_id": "UNKNOWN:0001",
  "term_label": "Unknown molecular function"
}